{
  "gene_symbol": "RYR2",
  "term_id": "GO:0030018",
  "gene": "UniProtKB:Q92736",
  "gene_name": "Ryanodine receptor 2",
  "term_label": "Z disc"
}